paraxial mesoderm structural organization [GO:0048352] (biological process) Also known as: paraxial mesoderm structural organisation Sources: GOC:dgh Definition: The process that contributes to the act of creating the structural organization of the paraxial mesoderm. This process pertains to the physical shaping of a rudimentary structure. Relationships: is_a mesoderm structural organization [GO:0048338]; is part of paraxial mesoderm morphogenesis [GO:0048340]